linear 1,3-beta-D-glucan synthase activity [GO:0140753] (molecular function) Relationships: is a type of 1,3-beta-D-glucan synthase activity [GO:0003843] Definition: Catalysis of the reaction: UDP-glucose + [(1->3)-beta-D-glucosyl](n) = UDP + a linear [(1->3)-beta-D-glucosyl](n+1). References: PMID:34959732